prunasin beta-glucosidase activity [GO:0050224] (molecular function) Sources: EC:3.2.1.118, RHEA:16489 Relationships: is a type of beta-glucosidase activity [GO:0008422] Definition: Catalysis of the reaction: (R)-prunasin + H2O = D-glucose + mandelonitrile. Also known as: prunasin b-glucosidase activity, prunasin beta-D-glucohydrolase activity, prunasin hydrolase activity